protein tyrosine kinase inhibitor activity [GO:0030292] (molecular function) Sources: GOC:mah Subtypes: transmembrane receptor protein tyrosine kinase inhibitor activity [GO:0030293], receptor signaling protein tyrosine kinase inhibitor activity [GO:0030294] Definition: Stops, prevents or reduces the activity of a protein tyrosine kinase. Relationships: is a type of protein kinase inhibitor activity [GO:0004860]; negatively regulates protein tyrosine kinase activity [GO:0004713]